{
  "gene": "UniProtKB:Q9UBL3",
  "gene_symbol": "ASH2L",
  "term_label": "Set1C/COMPASS complex",
  "gene_name": "Set1_Ash2 histone methyltransferase complex subunit ASH2",
  "term_id": "GO:0048188"
}